{
  "term_id": "GO:0005615",
  "term_label": "extracellular space",
  "gene": "UniProtKB:O00144",
  "gene_name": "Frizzled-9",
  "gene_symbol": "FZD9"
}